{
  "term_label": "cell surface",
  "gene_symbol": "ANTXR2",
  "gene": "UniProtKB:P58335",
  "term_id": "GO:0009986",
  "gene_name": "Anthrax toxin receptor 2"
}